cell trailing edge [GO:0031254] (cellular component) Sources: GOC:pg Also known as: back of cell, trailing edge Relationships: is a type of cellular anatomical structure [GO:0110165] Definition: The area of a motile cell opposite to the direction of movement.